negative regulation of neutrophil apoptotic process [GO:0033030] (biological process) Also known as: down regulation of neutrophil apoptosis, down-regulation of neutrophil apoptosis, downregulation of neutrophil apoptosis, inhibition of neutrophil apoptosis, negative regulation of neutrophil apoptosis Definition: Any process that stops, prevents, or reduces the frequency, rate, or extent of neutrophil apoptotic process. Sources: GOC:add, GOC:mtg_apoptosis Relationships: is_a regulation of neutrophil apoptotic process [GO:0033029]; is a type of negative regulation of myeloid cell apoptotic process [GO:0033033]; is a type of negative regulation of leukocyte apoptotic process [GO:2000107]; negatively regulates neutrophil apoptotic process [GO:0001781]